{
  "gene_symbol": "FAM219A",
  "gene_name": "Protein FAM219A",
  "gene": "UniProtKB:Q8IW50",
  "term_label": "Unknown cellular component",
  "term_id": "UNKNOWN:0003"
}